platelet alpha granule membrane [GO:0031092] (cellular component) Also known as: platelet alpha-granule membrane References: PMID:8467233 Sources: GOC:mah Definition: The lipid bilayer surrounding the platelet alpha granule. Relationships: is a type of secretory granule membrane [GO:0030667]; is part of platelet alpha granule [GO:0031091]